6-aminohexanoate-dimer hydrolase activity [GO:0019875] (molecular function) Sources: EC:3.5.1.46 Also known as: 6-aminohexanoic acid oligomer hydrolase activity, N-(6-aminohexanoyl)-6-aminohexanoate amidohydrolase activity Relationships: is a type of hydrolase activity, acting on carbon-nitrogen (but not peptide) bonds, in linear amides [GO:0016811] Definition: Catalysis of the reaction: N-(6-aminohexanoyl)-6-aminohexanoate + H2O = 2 6-aminohexanoate.